{
  "gene_name": "Acetylcholine receptor subunit alpha",
  "gene_symbol": "CHRNA1",
  "gene": "UniProtKB:P02708",
  "term_label": "membrane depolarization",
  "term_id": "GO:0051899"
}